diiodotyrosine transaminase activity [GO:0047861] (molecular function) Also known as: diiodotyrosine aminotransferase activity, 3,5-diiodo-L-tyrosine:2-oxoglutarate aminotransferase activity, halogenated tyrosine aminotransferase activity, halogenated tyrosine transaminase activity Relationships: is_a GO:0008483 Sources: EC:2.6.1.24, RHEA:19781 Definition: Catalysis of the reaction: 2-oxoglutarate + 3,5-diiodo-L-tyrosine = 3-(3,5-diiodo-4-hydroxyphenyl)pyruvate + L-glutamate.